{
  "gene_name": "ATP-sensitive inward rectifier potassium channel 14",
  "gene": "UniProtKB:Q9UNX9",
  "term_id": "GO:0005886",
  "gene_symbol": "KCNJ14",
  "term_label": "plasma membrane"
}